{
  "gene_name": "Guanine nucleotide-binding protein subunit beta-4",
  "term_label": "heterotrimeric G-protein complex",
  "term_id": "GO:0005834",
  "gene_symbol": "GNB4",
  "gene": "UniProtKB:Q9HAV0"
}